{
  "gene_symbol": "TH",
  "gene": "UniProtKB:P07101",
  "gene_name": "Tyrosine 3-monooxygenase",
  "term_id": "GO:0042418",
  "term_label": "epinephrine biosynthetic process"
}